negative regulation of cardiac endothelial to mesenchymal transition [GO:0062001] (biological process) References: PMID:26857067 Sources: GOC:BHF, GOC:BHF_miRNA, GOC:rph Definition: Any process that stops, prevents, or reduces the frequency, rate or extent of cardiac endothelial to mesenchymal transition. Relationships: is a type of negative regulation of cell differentiation [GO:0045596]; is a type of GO:0051241; is a type of regulation of cardiac endothelial to mesenchymal transition [GO:0061999]; negatively regulates cardiac endothelial to mesenchymal transition [GO:0140074]